{
  "gene_name": "U6 snRNA-associated Sm-like protein LSm4",
  "gene": "UniProtKB:Q9Y4Z0",
  "gene_symbol": "LSM4",
  "term_label": "spliceosomal tri-snRNP complex",
  "term_id": "GO:0097526"
}